zeaxanthin catabolic process [GO:1901826] (biological process) Also known as: zeaxanthin breakdown, zeaxanthin catabolism, zeaxanthin degradation Relationships: is a type of GO:0016124 Definition: The chemical reactions and pathways resulting in the breakdown of zeaxanthin. Sources: GOC:TermGenie, GOC:yaf, MetaCyc:PWY-5944, UniPathway:UPA00843